{
  "term_id": "GO:0006401",
  "gene": "UniProtKB:Q9BXU1",
  "term_label": "RNA catabolic process",
  "gene_symbol": "STK31",
  "gene_name": "Serine_threonine-protein kinase 31"
}